drought recovery [GO:0009819] (biological process) Definition: Any process that results in a change in state or activity of a cell or an organism (in terms of movement, secretion, enzyme production, gene expression, etc.) as a result of prolonged deprivation of water that restores that organism to a normal (non-stressed) condition. Also known as: drought tolerance Sources: GOC:lr Relationships: is a type of response to water deprivation [GO:0009414]